{
  "gene": "UniProtKB:Q13239",
  "term_id": "GO:0005737",
  "term_label": "cytoplasm",
  "gene_symbol": "SLA",
  "gene_name": "Src-like-adapter"
}